{
  "gene": "UniProtKB:Q9H963",
  "gene_name": "Putative zinc finger protein 702",
  "term_id": "UNKNOWN:0002",
  "term_label": "Unknown biological process",
  "gene_symbol": "ZNF702P"
}